{
  "term_label": "serine-type endopeptidase activity",
  "term_id": "GO:0004252",
  "gene": "UniProtKB:Q7RTY5",
  "gene_symbol": "PRSS48",
  "gene_name": "Serine protease 48"
}